{
  "term_label": "nucleus",
  "gene": "UniProtKB:P04733",
  "term_id": "GO:0005634",
  "gene_name": "Metallothionein-1F",
  "gene_symbol": "MT1F"
}